{
  "gene": "UniProtKB:E7ERA6",
  "gene_name": "RING finger protein 223",
  "gene_symbol": "RNF223",
  "term_id": "UNKNOWN:0003",
  "term_label": "Unknown cellular component"
}